flavin adenine dinucleotide catabolic process [GO:0072389] (biological process) Relationships: is_a nucleotide catabolic process [GO:0009166]; is a type of flavin-containing compound catabolic process [GO:0042728]; is a type of flavin adenine dinucleotide metabolic process [GO:0072387] Sources: GOC:mah Definition: The chemical reactions and pathways resulting in the breakdown of flavin adenine dinucleotide, which acts as a coenzyme or prosthetic group of various flavoprotein oxidoreductase enzymes. Also known as: FAD or FADH2 catabolic process, flavin adenine dinucleotide breakdown, flavin adenine dinucleotide catabolism, flavin adenine dinucleotide degradation